{
  "term_label": "membrane",
  "term_id": "GO:0016020",
  "gene_symbol": "ELAPOR2",
  "gene_name": "Endosome_lysosome-associated apoptosis and autophagy regulator family member 2",
  "gene": "UniProtKB:A8MWY0"
}